{
  "term_label": "extracellular space",
  "gene": "UniProtKB:Q7Z5A4",
  "term_id": "GO:0005615",
  "gene_symbol": "PRSS42P",
  "gene_name": "Putative serine protease 42"
}